{
  "term_id": "GO:0034553",
  "gene": "UniProtKB:Q5VUM1",
  "term_label": "mitochondrial respiratory chain complex II assembly",
  "gene_symbol": "SDHAF4",
  "gene_name": "Succinate dehydrogenase assembly factor 4, mitochondrial"
}